antigen processing and presentation of endogenous peptide antigen via MHC class I [GO:0019885] (biological process) Relationships: is a type of GO:0002474; is_a GO:0002483 Subtypes: antigen processing and presentation of endogenous peptide antigen via MHC class I via ER pathway [GO:0002484], GO:0002487 References: PMID:15771591 Sources: GOC:add, ISBN:0781735149 Definition: The process in which an antigen-presenting cell expresses a peptide antigen of endogenous origin on its cell surface in association with an MHC class I protein complex. The peptide antigen is typically, but not always, processed from a whole protein. Class I here refers to classical class I molecules. Also known as: antigen presentation, endogenous peptide antigen, antigen processing, endogenous antigen via MHC class I, antigen processing, endogenous antigen via major histocompatibility complex class I, endogenous peptide antigen processing and presentation via MHC class I Regulation: regulated by GO:1904282; negatively regulated by negative regulation of antigen processing and presentation of endogenous peptide antigen via MHC class I [GO:1904283]; RO_0002213 by positive regulation of antigen processing and presentation of endogenous peptide antigen via MHC class I [GO:1904284]